{
  "term_id": "GO:0005085",
  "gene_symbol": "PSD2",
  "gene_name": "PH and SEC7 domain-containing protein 2",
  "gene": "UniProtKB:Q9BQI7",
  "term_label": "guanyl-nucleotide exchange factor activity"
}